{
  "gene_name": "Teneurin-3",
  "gene_symbol": "TENM3",
  "gene": "UniProtKB:Q9P273",
  "term_label": "cell adhesion molecule binding",
  "term_id": "GO:0050839"
}